{
  "gene_name": "Secreted frizzled-related protein 3",
  "gene": "UniProtKB:Q92765",
  "gene_symbol": "FRZB",
  "term_label": "cytoplasm",
  "term_id": "GO:0005737"
}